replication fork progression beyond termination site [GO:0097046] (BP) Relationships: is_a regulation of DNA replication termination [GO:2000621] References: PMID:20797631 Sources: GOC:bf, GOC:mcc, GOC:pr Definition: Regulation of DNA replication by a mechanism that allows a DNA replication fork to progress beyond a termination site, which is a region containing fork pausing elements that influence the progression and merging of DNA replication forks.